regulation of apical constriction involved in ventral furrow formation [GO:0110073] (biological process) Definition: Any process that modulates the frequency, rate or extent of apical constriction involved in ventral furrow formation. References: PMID:28495958 Sources: GOC:ha Relationships: is a type of GO:0010470; is a type of regulation of cell morphogenesis [GO:0022604]; is a type of GO:1903115; regulates apical constriction involved in ventral furrow formation [GO:0110072] Subtypes: positive regulation of apical constriction involved in ventral furrow formation [GO:0110074]